{
  "gene_name": "Zinc transporter 6",
  "gene": "UniProtKB:Q6NXT4",
  "term_id": "UNKNOWN:0001",
  "term_label": "Unknown molecular function",
  "gene_symbol": "SLC30A6"
}